{
  "gene_name": "SLIT and NTRK-like protein 1",
  "gene_symbol": "SLITRK1",
  "term_label": "glutamatergic synapse",
  "term_id": "GO:0098978",
  "gene": "UniProtKB:Q96PX8"
}